{
  "gene_name": "Alpha-N-acetylgalactosaminide alpha-2,6-sialyltransferase 1",
  "term_id": "GO:0009312",
  "gene_symbol": "ST6GALNAC1",
  "gene": "UniProtKB:Q9NSC7",
  "term_label": "oligosaccharide biosynthetic process"
}